positive regulation of lymphocyte anergy [GO:0002913] (biological process) Relationships: is a type of positive regulation of tolerance induction [GO:0002645]; is a type of GO:0002911; positively regulates lymphocyte anergy [GO:0002249] Sources: GOC:add Also known as: up regulation of lymphocyte anergy, up-regulation of lymphocyte anergy, upregulation of lymphocyte anergy, activation of lymphocyte anergy, stimulation of lymphocyte anergy Subtypes: positive regulation of T cell anergy [GO:0002669], positive regulation of B cell anergy [GO:0002672] Definition: Any process that activates or increases the frequency, rate, or extent of lymphocyte anergy.